polynucleotide 3'-phosphatase activity [GO:0046403] (molecular function) Also known as: 2'(3')-polynucleotidase activity, 5'-polynucleotidekinase 3'-phosphatase activity, DNA 3'-phosphatase activity, deoxyribonucleate 3'-phosphatase activity, polynucleotide 3'-phosphohydrolase activity Sources: RHEA:14113 Definition: Catalysis of the reaction: a 3'end (2'-deoxyribonucleotide 3'-phosphate)-DNA + H2O = a 3'-end 2'-deoxyribonucleotide-DNA + phosphate. Relationships: is a type of phosphatase activity [GO:0016791]